{
  "term_id": "GO:0071962",
  "term_label": "mitotic sister chromatid cohesion, centromeric",
  "gene_name": "Shugoshin 1",
  "gene": "UniProtKB:Q5FBB7",
  "gene_symbol": "SGO1"
}